{
  "gene_symbol": "SPATA25",
  "gene_name": "Spermatogenesis-associated protein 25",
  "term_label": "Unknown cellular component",
  "term_id": "UNKNOWN:0003",
  "gene": "UniProtKB:Q9BR10"
}